{
  "gene_name": "Rho GTPase-activating protein 44",
  "gene": "UniProtKB:Q17R89",
  "term_label": "leading edge membrane",
  "term_id": "GO:0031256",
  "gene_symbol": "ARHGAP44"
}